depolarization of postsynaptic membrane [GO:0098819] (biological process) Sources: GOC:dos Definition: A process that depolarizes a postsynaptic membrane relative to its resting potential. This has an excitatory effect on the post-synaptic cell, moving the membrane potential towards the firing threshold. Relationships: is a type of regulation of postsynaptic membrane potential [GO:0060078]